{
  "gene_symbol": "COMT",
  "gene_name": "Catechol O-methyltransferase",
  "term_id": "GO:0042417",
  "term_label": "dopamine metabolic process",
  "gene": "UniProtKB:P21964"
}